negative regulation of lipid transport across blood-brain barrier [GO:1903001] (biological process) References: PMID:24345162 Sources: GOC:TermGenie, GOC:sjp, GO_REF:0000058 Definition: Any process that stops, prevents or reduces the frequency, rate or extent of lipid transport across blood-brain barrier. Also known as: down regulation of lipid transport across blood brain barrier, down-regulation of lipid transport across blood brain barrier, downregulation of lipid transport across blood brain barrier, negative regulation of lipid transport across blood brain barrier, inhibition of lipid transport across blood brain barrier Relationships: is a type of negative regulation of lipid transport [GO:0032369]; is a type of negative regulation of transport across blood-brain barrier [GO:0150202]; is a type of regulation of lipid transport across blood-brain barrier [GO:1903000]; negatively regulates GO:1990379